{
  "term_label": "Unknown molecular function",
  "gene_name": "Protein ZNF365",
  "gene_symbol": "ZNF365",
  "gene": "UniProtKB:Q70YC5",
  "term_id": "UNKNOWN:0001"
}